{
  "term_id": "GO:0000981",
  "gene_symbol": "ONECUT3",
  "gene_name": "One cut domain family member 3",
  "term_label": "DNA-binding transcription factor activity, RNA polymerase II-specific",
  "gene": "UniProtKB:O60422"
}